{
  "gene": "UniProtKB:P10124",
  "gene_name": "Serglycin",
  "gene_symbol": "SRGN",
  "term_label": "Unknown molecular function",
  "term_id": "UNKNOWN:0001"
}